{
  "term_id": "UNKNOWN:0001",
  "gene": "UniProtKB:A6NK53",
  "gene_symbol": "ZNF233",
  "term_label": "Unknown molecular function",
  "gene_name": "Zinc finger protein 233"
}